{
  "term_label": "phosphatidylinositol-mediated signaling",
  "gene_name": "1-phosphatidylinositol 4,5-bisphosphate phosphodiesterase beta-2",
  "gene": "UniProtKB:Q00722",
  "gene_symbol": "PLCB2",
  "term_id": "GO:0048015"
}